{
  "term_label": "alkylglycerophosphoethanolamine phosphodiesterase activity",
  "term_id": "GO:0047391",
  "gene_symbol": "ENPP2",
  "gene_name": "Ectonucleotide pyrophosphatase_phosphodiesterase family member 2",
  "gene": "UniProtKB:Q13822"
}